{
  "term_id": "UNKNOWN:0002",
  "gene_symbol": "ARHGAP11A",
  "gene_name": "Rho GTPase-activating protein 11A",
  "term_label": "Unknown biological process",
  "gene": "UniProtKB:Q6P4F7"
}